entry of bacterium into host cell [GO:0035635] (biological process) Definition: The process in which a bacterium enters a host cell. The host is defined as the larger of the organisms involved in a symbiotic interaction. References: PMID:21187937 Sources: GOC:bf Also known as: bacterial entry into host cell, invasion of bacteria into host cell Relationships: is a type of symbiont entry into host [GO:0044409] Regulation: RO_0002211 by regulation of entry of bacterium into host cell [GO:2000535]; negatively regulated by negative regulation of entry of bacterium into host cell [GO:2000536]